nuclear ubiquitin ligase complex [GO:0000152] (cellular component) Relationships: is a type of GO:0000151; is a type of nuclear protein-containing complex [GO:0140513] Definition: A ubiquitin ligase complex found in the nucleus. Subtypes: anaphase-promoting complex [GO:0005680], BRCA1-BARD1 complex [GO:0031436], SUMO-targeted ubiquitin ligase complex [GO:0033768], GO:0035102, nuclear SCF ubiquitin ligase complex [GO:0043224], CLRC complex [GO:0043494], GO:0097658, BCOR complex [GO:0140261] Sources: GOC:mah